{
  "gene_symbol": "NKX6-1",
  "gene_name": "Homeobox protein Nkx-6.1",
  "term_label": "RNA polymerase II cis-regulatory region sequence-specific DNA binding",
  "gene": "UniProtKB:P78426",
  "term_id": "GO:0000978"
}